{
  "term_id": "GO:0000398",
  "gene_symbol": "EIF4A3",
  "gene": "UniProtKB:P38919",
  "gene_name": "Eukaryotic initiation factor 4A-III",
  "term_label": "mRNA splicing, via spliceosome"
}